{
  "gene_name": "HLA class I histocompatibility antigen, B alpha chain",
  "term_label": "extracellular space",
  "term_id": "GO:0005615",
  "gene": "UniProtKB:P01889",
  "gene_symbol": "HLA-B"
}